pollen wall assembly [GO:0010208] (biological process) Relationships: is a type of GO:0010927; is a type of external encapsulating structure organization [GO:0045229]; is part of pollen development [GO:0009555] Definition: The formation of reticulate pollen wall pattern consisting of two layers, exine and intine. Also known as: pollen wall formation References: PMID:11743117 Subtypes: pollen exine formation [GO:0010584], pollen intine formation [GO:0160030]